{
  "term_id": "UNKNOWN:0003",
  "gene_symbol": "MUC20",
  "term_label": "Unknown cellular component",
  "gene_name": "Mucin-20",
  "gene": "UniProtKB:Q8N307"
}